centrosomal corona [GO:0031592] (cellular component) Sources: GOC:kp, GOC:mah Relationships: is a type of cellular anatomical structure [GO:0110165]; is part of centrosome [GO:0005813] Definition: An amorphous structure surrounding the core of the centrosome, from which microtubules are nucleated; contains gamma-tubulin. Note: Note that the centrosomal corona has been observed in Dictyostelium, and is the functional equivalent of pericentriolar material.